{
  "gene_symbol": "PPDPF",
  "term_id": "UNKNOWN:0002",
  "term_label": "Unknown biological process",
  "gene_name": "Pancreatic progenitor cell differentiation and proliferation factor",
  "gene": "UniProtKB:Q9H3Y8"
}